{
  "gene": "UniProtKB:Q9H6B9",
  "gene_name": "Epoxide hydrolase 3",
  "term_id": "UNKNOWN:0003",
  "gene_symbol": "EPHX3",
  "term_label": "Unknown cellular component"
}